{
  "term_label": "Unknown molecular function",
  "gene_symbol": "C1orf54",
  "term_id": "UNKNOWN:0001",
  "gene_name": "Uncharacterized protein C1orf54",
  "gene": "UniProtKB:Q8WWF1"
}